{
  "gene_symbol": "CXorf58",
  "term_id": "UNKNOWN:0002",
  "gene_name": "Uncharacterized protein CXorf58",
  "gene": "UniProtKB:Q96LI9",
  "term_label": "Unknown biological process"
}